{
  "term_id": "UNKNOWN:0002",
  "term_label": "Unknown biological process",
  "gene_name": "Methionine aminopeptidase 2",
  "gene": "UniProtKB:P50579",
  "gene_symbol": "METAP2"
}